{
  "gene_symbol": "ANKRD35",
  "term_id": "UNKNOWN:0003",
  "gene_name": "Ankyrin repeat domain-containing protein 35",
  "term_label": "Unknown cellular component",
  "gene": "UniProtKB:Q8N283"
}